L-alanine oxidation to pyruvate via D-alanine [GO:0019480] (biological process) Definition: The chemical reactions and pathways resulting in the breakdown of L-alanine to pyruvate, with D-alanine as an intermediate. Sources: MetaCyc:ALADEG-PWY Relationships: is a type of L-alanine catabolic process [GO:0042853]